{
  "term_label": "positive regulation of transcription by RNA polymerase II",
  "term_id": "GO:0045944",
  "gene_symbol": "HIPK2",
  "gene": "UniProtKB:Q9H2X6",
  "gene_name": "Homeodomain-interacting protein kinase 2"
}